{
  "term_label": "Unknown cellular component",
  "term_id": "UNKNOWN:0003",
  "gene": "UniProtKB:Q9HCN3",
  "gene_name": "Post-GPI attachment to proteins factor 6",
  "gene_symbol": "PGAP6"
}